{
  "term_id": "GO:0005634",
  "gene_name": "Paired mesoderm homeobox protein 2A",
  "gene": "UniProtKB:O14813",
  "gene_symbol": "PHOX2A",
  "term_label": "nucleus"
}